UDP phosphatase activity [GO:0045134] (molecular function) Sources: RHEA:64876 Definition: Catalysis of the reaction: UDP + H2O = UMP + phosphate. Also known as: UDP phosphohydrolase activity, uridine-diphosphatase activity, UDPase activity, uridine 5'-diphosphatase activity, uridine diphosphatase activity Relationships: is a type of nucleoside diphosphate phosphatase activity [GO:0017110]